epithelial cell migration involved in distal tubule morphogenesis [GO:0072157] (biological process) Definition: The orderly movement of epithelial cells within a renal tubule that contributes to distal tubule morphogenesis. Relationships: is a type of epithelial cell migration involved in nephron tubule morphogenesis [GO:0072155]; is part of distal tubule morphogenesis [GO:0072156] Sources: GOC:mtg_kidney_jan10 Subtypes: epithelial cell migration involved in mesonephric distal tubule morphogenesis [GO:0061279], epithelial cell migration involved in metanephric distal tubule morphogenesis [GO:0072291]